{
  "gene_symbol": "RAB3GAP1",
  "term_label": "brain development",
  "gene_name": "Rab3 GTPase-activating protein catalytic subunit",
  "term_id": "GO:0007420",
  "gene": "UniProtKB:Q15042"
}